negative regulation of direction of cell growth [GO:0061391] (biological process) Definition: Any process that decreases the direction of cell growth. Sources: GOC:mah, GOC:vw Relationships: is a type of negative regulation of cell growth [GO:0030308]; is a type of GO:0061389